{
  "gene_symbol": "TPRA1",
  "gene": "UniProtKB:Q86W33",
  "gene_name": "Transmembrane protein adipocyte-associated 1",
  "term_id": "GO:0007186",
  "term_label": "G protein-coupled receptor signaling pathway"
}